intermediate-density lipoprotein particle [GO:0034363] (CC) Relationships: is a type of triglyceride-rich plasma lipoprotein particle [GO:0034385] Definition: A triglyceride-rich lipoprotein particle that typically contains APOB100, APOE and APOCs and has a density of 1.006-1.019 g/ml and a diameter of between 25-30 nm. IDL particles are found in blood and are formed by the delipidation of very-low-density lipoprotein particles (VLDL). IDL particles are removed from blood by the liver, following binding to the APOE receptor, or are converted to low-density lipoprotein (LDL). Also known as: IDL complex, IDL particle, intermediate-density lipoprotein complex Sources: GOC:BHF, GOC:expert_pt, GOC:mah, GOC:rl